negative regulation of mesonephros development [GO:0061218] (biological process) Relationships: is a type of regulation of mesonephros development [GO:0061217]; is a type of negative regulation of kidney development [GO:0090185]; negatively regulates GO:0001823 Definition: Any process that decreases the rate, frequency or extent of mesonephros development. Mesonephros development is the process whose specific outcome is the progression of the mesonephros over time, from its formation to the mature structure. The mesonephros is an organ that filters the blood and excretes the end products of body metabolism in the form of urine. Sources: GOC:mtg_kidney_jan10 Subtypes: negative regulation of mesenchymal cell apoptotic process involved in mesonephric nephron morphogenesis [GO:0061296]